{
  "gene_symbol": "OR6M1",
  "term_id": "GO:0005886",
  "gene": "UniProtKB:Q8NGM8",
  "term_label": "plasma membrane",
  "gene_name": "Olfactory receptor 6M1"
}